calmodulin-dependent protein phosphatase activity [GO:0033192] (molecular function) References: PMID:15359118 Sources: GOC:mah Also known as: calcium- and calmodulin-dependent protein phosphatase activity, calcium/calmodulin-dependent protein phosphatase activity, calcineurin activity, Ca2+/CaM-dependent protein phosphatase activity Relationships: is a type of GO:0004723 Definition: Catalysis of the reaction: protein serine/threonine phosphate + H2O = protein serine/threonine + phosphate, dependent on the presence of calcium-bound calmodulin.